{
  "term_label": "plasma membrane",
  "gene": "UniProtKB:Q9H2S1",
  "gene_name": "Small conductance calcium-activated potassium channel protein 2",
  "term_id": "GO:0005886",
  "gene_symbol": "KCNN2"
}